homomethionine N-monooxygenase activity [GO:0120526] (molecular function) Sources: RHEA:51972 Relationships: is a type of GO:0016712 Definition: Catalysis of the reaction: an L-polyhomomethionine + 2 O2 + 2 reduced [NADPH--hemoprotein reductase] = an (E)-omega-(methylsulfanyl)-alkanal oxime + CO2 + 2 H(+) + 3 H2O + 2 oxidized [NADPH--hemoprotein reductase].